{
  "term_label": "cell adhesion molecule binding",
  "term_id": "GO:0050839",
  "gene_name": "Protocadherin beta-6",
  "gene": "UniProtKB:Q9Y5E3",
  "gene_symbol": "PCDHB6"
}